curcumin catabolic process [GO:0036040] (biological process) Definition: The chemical reactions and pathways resulting in the breakdown of the polyphenol, curcumin. Also known as: (1E,6E)-1,7-bis(4-hydroxy-3-methoxyphenyl)hepta-1,6-diene-3,5-dione breakdown, (1E,6E)-1,7-bis(4-hydroxy-3-methoxyphenyl)hepta-1,6-diene-3,5-dione catabolic process, (1E,6E)-1,7-bis(4-hydroxy-3-methoxyphenyl)hepta-1,6-diene-3,5-dione catabolism, (1E,6E)-1,7-bis(4-hydroxy-3-methoxyphenyl)hepta-1,6-diene-3,5-dione degradation, curcumin breakdown, curcumin catabolism, curcumin degradation, diferuloylmethane breakdown, diferuloylmethane catabolic process, diferuloylmethane catabolism, diferuloylmethane degradation, turmeric yellow breakdown, turmeric yellow catabolic process, turmeric yellow catabolism, turmeric yellow degradation Relationships: is a type of GO:0019336; is_a ketone catabolic process [GO:0042182]; is a type of olefinic compound catabolic process [GO:0120256]; is a type of ether catabolic process [GO:1901502] References: PMID:21467222